{
  "gene_symbol": "OR2T7",
  "term_id": "GO:0050911",
  "gene": "UniProtKB:P0C7T2",
  "gene_name": "Olfactory receptor 2T7",
  "term_label": "detection of chemical stimulus involved in sensory perception of smell"
}